negative regulation of phosphatidylserine exposure on apoptotic cell surface [GO:1905781] (biological process) References: PMID:17401362 Sources: GOC:TermGenie, GOC:kmv, GO_REF:0000058 Definition: Any process that stops, prevents or reduces the frequency, rate or extent of phosphatidylserine exposure on apoptotic cell surface. Also known as: down regulation of externalization of phosphatidylserine, down regulation of phosphatidylserine exposure on apoptotic cell surface, down-regulation of externalization of phosphatidylserine, down-regulation of phosphatidylserine exposure on apoptotic cell surface, downregulation of externalization of phosphatidylserine, downregulation of phosphatidylserine exposure on apoptotic cell surface, negative regulation of externalization of phosphatidylserine, inhibition of externalization of phosphatidylserine, inhibition of phosphatidylserine exposure on apoptotic cell surface Relationships: is a type of negative regulation of phospholipid translocation [GO:0061093]; is a type of negative regulation of execution phase of apoptosis [GO:1900118]; is a type of regulation of phosphatidylserine exposure on apoptotic cell surface [GO:1905780]; negatively regulates phosphatidylserine exposure on apoptotic cell surface [GO:0070782]